{
  "gene_name": "Phosphoenolpyruvate carboxykinase, cytosolic [GTP]",
  "gene_symbol": "PCK1",
  "term_id": "GO:0070365",
  "term_label": "hepatocyte differentiation",
  "gene": "UniProtKB:P35558"
}